{
  "gene": "UniProtKB:Q13098",
  "term_label": "COP9 signalosome",
  "gene_name": "COP9 signalosome complex subunit 1",
  "gene_symbol": "GPS1",
  "term_id": "GO:0008180"
}